{
  "gene_symbol": "PPCDC",
  "term_id": "GO:0071513",
  "gene": "UniProtKB:Q96CD2",
  "gene_name": "Phosphopantothenoylcysteine decarboxylase",
  "term_label": "phosphopantothenoylcysteine decarboxylase complex"
}